{
  "term_id": "UNKNOWN:0002",
  "term_label": "Unknown biological process",
  "gene_name": "KH homology domain-containing protein 1",
  "gene_symbol": "KHDC1",
  "gene": "UniProtKB:Q4VXA5"
}